{
  "gene": "UniProtKB:Q9H7U1",
  "gene_name": "Serine-rich coiled-coil domain-containing protein 2",
  "term_id": "GO:0001578",
  "gene_symbol": "CCSER2",
  "term_label": "microtubule bundle formation"
}